regulation of cellular pH [GO:0030641] (biological process) Sources: GOC:dph, GOC:mah, GOC:tb Relationships: is a type of regulation of pH [GO:0006885]; is a type of GO:0030003 Definition: Any process involved in the maintenance of an internal equilibrium of hydrogen ions (protons) within a cell or between a cell and its external environment. Also known as: cellular hydrogen ion homeostasis, proton homeostasis Subtypes: regulation of intracellular pH [GO:0051453]